steroid hormone aporeceptor complex [GO:0005831] (cellular component) Relationships: is a type of protein-containing complex [GO:0032991]; is part of GO:0005829 References: PMID:7493981 Definition: A protein complex consisting of a steroid receptor associated with nonreceptor proteins, minimally a dimer of Hsp90 and a monomer of hsp56/FKBP59; forms in the absence of bound ligand.